{
  "gene": "UniProtKB:P11908",
  "term_id": "GO:0004749",
  "gene_name": "Ribose-phosphate pyrophosphokinase 2",
  "term_label": "ribose phosphate diphosphokinase activity",
  "gene_symbol": "PRPS2"
}